{
  "term_id": "UNKNOWN:0001",
  "gene_symbol": "A0A0G2JQZ4",
  "term_label": "Unknown molecular function",
  "gene": "UniProtKB:A0A0G2JQZ4",
  "gene_name": "Uncharacterized protein"
}